{
  "term_id": "UNKNOWN:0003",
  "term_label": "Unknown cellular component",
  "gene": "UniProtKB:P57727",
  "gene_symbol": "TMPRSS3",
  "gene_name": "Transmembrane protease serine 3"
}